{
  "gene": "UniProtKB:A4D250",
  "gene_name": "B-cell acute lymphoblastic leukemia-expressed protein",
  "term_label": "Unknown biological process",
  "term_id": "UNKNOWN:0002",
  "gene_symbol": "BLACE"
}